{
  "gene": "UniProtKB:Q8IX12",
  "gene_symbol": "CCAR1",
  "term_id": "UNKNOWN:0001",
  "gene_name": "Cell division cycle and apoptosis regulator protein 1",
  "term_label": "Unknown molecular function"
}